{
  "gene_name": "Transmembrane protein 119",
  "term_label": "positive regulation of osteoblast differentiation",
  "gene": "UniProtKB:Q4V9L6",
  "term_id": "GO:0045669",
  "gene_symbol": "TMEM119"
}